{
  "term_id": "GO:0002951",
  "gene_symbol": "GGT5",
  "gene": "UniProtKB:P36269",
  "gene_name": "Glutathione hydrolase 5 proenzyme",
  "term_label": "leukotriene-C(4) hydrolase"
}